ditrans,polycis-undecaprenyl-diphosphate synthase [(2E,6E)-farnesyl-diphosphate specific] activity [GO:0008834] (molecular function) Also known as: di-trans,poly-cis-decaprenylcistransferase activity, di-trans,poly-cis-undecaprenyl-diphosphate synthase activity, undecaprenyl diphosphate synthase activity, UPP synthetase activity, bactoprenyl-diphosphate synthase activity, di-trans,poly-cis-decaprenyl-diphosphate:isopentenyl-diphosphate undecaprenylcistransferase activity, undecaprenyl diphosphate synthetase activity, undecaprenyl pyrophosphate synthase activity, undecaprenyl pyrophosphate synthetase activity, undecaprenyl-diphosphate synthase activity Definition: Catalysis of the reaction: (2E,6E)-farnesyl diphosphate + 8 isopentenyl diphosphate = di-trans,octa-cis-undecaprenyl diphosphate + 8 diphosphate. Relationships: is a type of ditrans,polycis-polyprenyl diphosphate synthase [(2E,6E)-farnesyl diphosphate specific] activity [GO:0045547] Sources: RHEA:27551